{
  "gene": "UniProtKB:Q8N5I3",
  "term_label": "endoplasmic reticulum",
  "gene_name": "Potassium channel regulatory protein",
  "gene_symbol": "KCNRG",
  "term_id": "GO:0005783"
}